{
  "gene_name": "HLA class II histocompatibility antigen, DRB1 beta chain",
  "term_label": "lysosomal membrane",
  "gene": "UniProtKB:P01911",
  "gene_symbol": "HLA-DRB1",
  "term_id": "GO:0005765"
}